isoprenoid binding [GO:0019840] (molecular function) Definition: Binding to an isoprenoid compound, isoprene (2-methylbuta-1,3-diene) or compounds containing or derived from linked isoprene (3-methyl-2-butenylene) residues. Relationships: is a type of lipid binding [GO:0008289] Sources: GOC:jl Subtypes: juvenile hormone binding [GO:0005500], retinoid binding [GO:0005501], gibberellin binding [GO:0010331], abscisic acid binding [GO:0010427], xanthophyll binding [GO:0051738]